phthiocerol biosynthetic process [GO:0097040] (biological process) Relationships: is a type of lipid biosynthetic process [GO:0008610]; is a type of glycol biosynthetic process [GO:0042845] References: PMID:9201977 Sources: GOC:dph, GOC:ecd Also known as: phthiocerol anabolism, phthiocerol biosynthesis, phthiocerol formation, phthiocerol synthesis Definition: The chemical reactions and pathways resulting in the formation of phthiocerol, a lipid-based 1,3-glycol consisting of (3S,4R)-3-methoxy-4-methylnonacosane having (9R)- and (11S)-hydroxy substituents.